{
  "gene_symbol": "COL22A1",
  "gene_name": "Collagen alpha-1(XXII) chain",
  "term_label": "extracellular matrix organization",
  "gene": "UniProtKB:Q8NFW1",
  "term_id": "GO:0030198"
}